ADP-ribosylarginine hydrolase activity [GO:0003875] (molecular function) Relationships: is a type of GO:0016799; is a type of catalytic activity, acting on a protein [GO:0140096] Also known as: ADPribosylarginine hydrolase activity, ADP-ribose-L-arginine cleavage enzyme activity, ADP-ribose-L-arginine cleaving enzyme activity, N(omega)-(ADP-D-ribosyl)-L-arginine ADP-ribosylhydrolase activity, nomega-(ADP-D-ribosyl)-L-arginine ADP-ribosylhydrolase activity, omega-protein-N-(ADP-D-ribosyl)-L-arginine ADP-ribosylhydrolase activity, protein ADP-ribosylarginine hydrolase activity, protein-nomega-(ADP-D-ribosyl)-L-arginine ADP-ribosylhydrolase activity Definition: Catalysis of the reactions: H2O + N(omega)-(ADP-D-ribosyl)-L-arginyl-[protein] = ADP-D-ribose + L-arginyl-[protein], and H2O + N(omega)-(ADP-D-ribosyl)-L-arginine = ADP-D-ribose + L-arginine. Sources: EC:3.2.2.19